D-ribose pyranase activity [GO:0062193] (molecular function) Definition: Catalysis of the reactions: beta-D-ribopyranose = beta-D-ribofuranose, and beta-allofuranose = beta-allopyranose. Relationships: is a type of intramolecular transferase activity [GO:0016866] Sources: EC:5.4.99.62